{
  "gene_name": "Nephrocystin-4",
  "gene_symbol": "NPHP4",
  "gene": "UniProtKB:O75161",
  "term_label": "ciliary base",
  "term_id": "GO:0097546"
}